{
  "gene_name": "Uncharacterized protein C15orf62, mitochondrial",
  "term_label": "regulation of cell shape",
  "gene_symbol": "C15orf62",
  "term_id": "GO:0008360",
  "gene": "UniProtKB:A8K5M9"
}